{
  "gene_name": "E3 ubiquitin-protein ligase CBL",
  "gene": "UniProtKB:P22681",
  "gene_symbol": "CBL",
  "term_id": "GO:0030971",
  "term_label": "receptor tyrosine kinase binding"
}